{
  "term_label": "Unknown biological process",
  "gene_symbol": "MS4A4E",
  "term_id": "UNKNOWN:0002",
  "gene": "UniProtKB:Q96PG1",
  "gene_name": "Putative membrane-spanning 4-domains subfamily A member 4E"
}